R-loop processing [GO:0062176] (biological process) Relationships: is a type of chromatin remodeling [GO:0006338] Definition: A DNA metabolic process that results in the disassembly of R-loops. R-loops are three-stranded nucleic acid structures consisitng of an RNA:DNA heteroduplex and a looped-out non-template strand. Aberrant formation and persistence of R-loops block transcription elongation and cause DNA damage. Mechanisms that resolve R-loops are essential for genome stability. Also known as: R-loop disassembly References: PMID:27252122, PMID:28790157, PMID:33986538